{
  "term_label": "recycling endosome",
  "gene_symbol": "WIPF3",
  "gene": "UniProtKB:A6NGB9",
  "gene_name": "WAS_WASL-interacting protein family member 3",
  "term_id": "GO:0055037"
}